positive regulation of homotypic cell-cell adhesion [GO:0034112] (BP) Sources: GOC:add Relationships: is a type of positive regulation of cell-cell adhesion [GO:0022409]; is a type of regulation of homotypic cell-cell adhesion [GO:0034110]; positively regulates homotypic cell-cell adhesion [GO:0034109] Subtypes: positive regulation of erythrocyte aggregation [GO:0034120], positive regulation of platelet aggregation [GO:1901731] Definition: Any process that activates or increases the frequency, rate, or extent of homotypic cell-cell adhesion.